{
  "term_id": "GO:0005911",
  "gene": "UniProtKB:Q7Z4I7",
  "gene_symbol": "LIMS2",
  "gene_name": "LIM and senescent cell antigen-like-containing domain protein 2",
  "term_label": "cell-cell junction"
}